{
  "term_label": "U2 snRNP",
  "gene": "UniProtKB:P62308",
  "term_id": "GO:0005686",
  "gene_name": "Small nuclear ribonucleoprotein G",
  "gene_symbol": "SNRPG"
}